{
  "term_label": "mRNA splicing, via spliceosome",
  "gene_symbol": "ZCRB1",
  "gene_name": "Zinc finger CCHC-type and RNA-binding motif-containing protein 1",
  "gene": "UniProtKB:Q8TBF4",
  "term_id": "GO:0000398"
}